{
  "term_id": "GO:0045216",
  "term_label": "cell-cell junction organization",
  "gene_symbol": "LIMS1",
  "gene": "UniProtKB:P48059",
  "gene_name": "LIM and senescent cell antigen-like-containing domain protein 1"
}